{
  "term_label": "beta-carotene 15,15'-dioxygenase activity",
  "gene_name": "Beta,beta-carotene 15,15'-dioxygenase",
  "gene_symbol": "BCO1",
  "gene": "UniProtKB:Q9HAY6",
  "term_id": "GO:0003834"
}